{
  "gene_name": "Heat shock protein beta-8",
  "gene_symbol": "HSPB8",
  "gene": "UniProtKB:Q9UJY1",
  "term_id": "GO:0101031",
  "term_label": "protein folding chaperone complex"
}